protein dephosphorylation [GO:0006470] (biological process) Relationships: is a type of dephosphorylation [GO:0016311]; is a type of protein modification process [GO:0036211] Subtypes: peptidyl-tyrosine dephosphorylation [GO:0035335], GO:0035970, peptidyl-histidine dephosphorylation [GO:0035971], regulation of translational initiation by eIF2 alpha dephosphorylation [GO:0036496], peptidyl-serine dephosphorylation [GO:0070262], GO:0098628 Also known as: protein amino acid dephosphorylation Sources: GOC:hb Definition: The process of removing one or more phosphoric residues from a protein.